{
  "gene_symbol": "NLRP13",
  "gene_name": "NACHT, LRR and PYD domains-containing protein 13",
  "term_id": "GO:0005737",
  "term_label": "cytoplasm",
  "gene": "UniProtKB:Q86W25"
}